{
  "gene_symbol": "TLX1NB",
  "term_label": "Unknown cellular component",
  "gene_name": "Putative TLX1 neighbor protein",
  "term_id": "UNKNOWN:0003",
  "gene": "UniProtKB:P0CAT3"
}